sepiapterin reductase (NADP+) activity [GO:0004757] (molecular function) Also known as: 7,8-dihydrobiopterin:NADP+ oxidoreductase activity Definition: Catalysis of the reactions: 7,8-dihydrobiopterin + NADP+ = sepiapterin + NADPH + H+ and (6R)-L-erythro-5,6,7,8-tetrahydrobiopterin + 2 NADP+ = 6-pyruvoyl-5,6,7,8-tetrahydropterin + 2 H+ + 2 NADPH. Relationships: is a type of oxidoreductase activity, acting on the CH-OH group of donors, NAD or NADP as acceptor [GO:0016616] Sources: EC:1.1.1.153